L-alanine:2-oxoglutarate aminotransferase activity [GO:0004021] (molecular function) Sources: RHEA:19453 Note: Note that this term has a MetaCyc pathway reference as the pathway only has a single step. Also known as: L-alanine aminotransferase activity, L-alanine transaminase activity, alanine aminotransferase activity, alanine transaminase activity, beta-alanine aminotransferase, pyruvate transaminase activity, ALT, GPT, L-alanine-alpha-ketoglutarate aminotransferase activity, alanine-alpha-ketoglutarate aminotransferase activity, alanine-pyruvate aminotransferase activity, glutamic acid-pyruvic acid transaminase activity, glutamic--alanine transaminase activity, glutamic--pyruvic transaminase activity, glutamic-pyruvic aminotransferase activity, pyruvate-alanine aminotransferase activity, pyruvate-glutamate transaminase activity Definition: Catalysis of the reaction: 2-oxoglutarate + L-alanine = L-glutamate + pyruvate. Relationships: is a type of alanine-oxo-acid transaminase activity [GO:0047635]